{
  "gene": "UniProtKB:Q13322",
  "term_label": "Unknown cellular component",
  "term_id": "UNKNOWN:0003",
  "gene_name": "Growth factor receptor-bound protein 10",
  "gene_symbol": "GRB10"
}